{
  "term_label": "transcription factor TFIID complex",
  "gene_name": "Transcription initiation factor TFIID subunit 3",
  "term_id": "GO:0005669",
  "gene_symbol": "TAF3",
  "gene": "UniProtKB:Q5VWG9"
}